spermidine transmembrane transport [GO:1903711] (biological process) Relationships: is a type of GO:0015848; is a type of polyamine transmembrane transport [GO:1902047] Subtypes: GO:0140203 References: PMID:15637075 Sources: GOC:TermGenie, GO_REF:0000069 Definition: The process in which spermidine is transported across a membrane.